{
  "term_label": "regulation of transcription by RNA polymerase II",
  "gene": "UniProtKB:Q15940",
  "gene_name": "Putative zinc finger protein 726P1",
  "term_id": "GO:0006357",
  "gene_symbol": "ZNF726P1"
}